{
  "gene_symbol": "LHX8",
  "term_label": "DNA-binding transcription factor activity, RNA polymerase II-specific",
  "gene_name": "LIM_homeobox protein Lhx8",
  "term_id": "GO:0000981",
  "gene": "UniProtKB:Q68G74"
}